maternal behavior [GO:0042711] (biological process) Relationships: is a type of GO:0060746 Also known as: maternal behaviour Definition: Female behaviors associated with the care and rearing of offspring. Sources: GOC:curators